{
  "gene": "UniProtKB:P51959",
  "term_label": "G1/S transition of mitotic cell cycle",
  "gene_symbol": "CCNG1",
  "term_id": "GO:0000082",
  "gene_name": "Cyclin-G1"
}